protein prenylation [GO:0018342] (biological process) Also known as: protein amino acid prenylation, C-terminal protein prenylation Relationships: is a type of protein modification process [GO:0036211]; is a type of prenylation [GO:0097354] Subtypes: protein farnesylation [GO:0018343], GO:0018344 Definition: The covalent attachment of a prenyl group to a protein; geranyl, farnesyl, or geranylgeranyl groups may be added. Sources: GOC:di, ISBN:0198506732